{
  "term_label": "guanyl-nucleotide exchange factor activity",
  "gene_symbol": "RMC1",
  "gene_name": "Regulator of MON1-CCZ1 complex",
  "term_id": "GO:0005085",
  "gene": "UniProtKB:Q96DM3"
}